caudal ganglionic eminence cell proliferation [GO:0022021] (biological process) Relationships: is a type of subpallium cell proliferation in forebrain [GO:0022012] Definition: The multiplication or reproduction of caudal ganglionic eminence cells, resulting in the expansion of a cell population. Sources: GOC:cls, GOC:dgh, GOC:dph, GOC:jid, GO_REF:0000021